regulation of cardiac conduction [GO:1903779] (BP) Subtypes: regulation of atrial cardiac muscle cell action potential [GO:0098910], negative regulation of cardiac conduction [GO:1903780], positive regulation of cardiac conduction [GO:1903781] References: PMID:12967627 Sources: GOC:BHF, GOC:TermGenie, GOC:mtg_cardiac_conduct_nov11, GOC:rph, GO_REF:0000058 Definition: Any process that modulates the frequency, rate or extent of cardiac conduction. Relationships: is a type of GO:0008016; regulates cardiac conduction [GO:0061337]